{
  "gene": "UniProtKB:Q9NVP1",
  "term_id": "UNKNOWN:0001",
  "gene_symbol": "DDX18",
  "gene_name": "ATP-dependent RNA helicase DDX18",
  "term_label": "Unknown molecular function"
}